{
  "gene_name": "Elongator complex protein 3",
  "term_label": "Unknown molecular function",
  "term_id": "UNKNOWN:0001",
  "gene_symbol": "ELP3",
  "gene": "UniProtKB:Q9H9T3"
}